regulation of filamentous growth of a population of unicellular organisms in response to pH [GO:1900741] (biological process) Relationships: is a type of regulation of response to stimulus [GO:0048583]; is_a regulation of filamentous growth of a population of unicellular organisms [GO:1900428]; regulates filamentous growth of a population of unicellular organisms in response to pH [GO:0036177] Definition: Any process that modulates the frequency, rate or extent of filamentous growth of a population of unicellular organisms in response to pH. Subtypes: regulation of filamentous growth of a population of unicellular organisms in response to neutral pH [GO:1900440], negative regulation of filamentous growth of a population of unicellular organisms in response to pH [GO:1900742], GO:1900743 Sources: GOC:TermGenie, GOC:di